{
  "gene": "UniProtKB:A6NI15",
  "term_label": "mesoderm formation",
  "term_id": "GO:0001707",
  "gene_symbol": "MSGN1",
  "gene_name": "Mesogenin-1"
}